negative regulation of hindgut contraction [GO:0060451] (biological process) Definition: Any process that decreases the frequency, rate or extent of muscle contraction of the hindgut, the posterior part of the alimentary canal, including the rectum, and the large intestine. Relationships: is a type of GO:0043134; is a type of negative regulation of smooth muscle contraction [GO:0045986]; is a type of negative regulation of digestive system process [GO:0060457]; negatively regulates GO:0043133 Sources: GOC:dph, GOC:tb